{
  "gene_name": "Tubulin beta-6 chain",
  "gene": "UniProtKB:Q9BUF5",
  "term_id": "GO:0000226",
  "term_label": "microtubule cytoskeleton organization",
  "gene_symbol": "TUBB6"
}